{
  "term_id": "GO:0005813",
  "gene_symbol": "CCDC88B",
  "gene": "UniProtKB:A6NC98",
  "gene_name": "Coiled-coil domain-containing protein 88B",
  "term_label": "centrosome"
}